pyrimidine-specific mismatch base pair DNA N-glycosylase activity [GO:0008263] (molecular function) Subtypes: G/U mismatch-specific uracil-DNA glycosylase activity [GO:0043739], GO:0141016 Definition: Catalysis of the removal of mismatched pyrimidine bases in DNA. Enzymes with this activity recognize and remove pyrimidines present in mismatches by cleaving the N-C1' glycosidic bond between the target damaged DNA base and the deoxyribose sugar. The reaction releases a free base and leaves an apyrimidinic (AP) site. Also known as: G/T-mismatch-specific thymine-DNA glycosylase activity Relationships: is a type of mismatch base pair DNA N-glycosylase activity [GO:0000700] References: PMID:9224623 Sources: GOC:elh